beta-alanine biosynthetic process via 3-hydroxypropionate [GO:0033395] (biological process) Definition: The chemical reactions and pathways resulting in the formation of beta-alanine via the intermediate 3-hydroxypropionate. Also known as: beta-alanine anabolism via 3-hydroxypropionate, beta-alanine biosynthesis via 3-hydroxypropionate, beta-alanine formation via 3-hydroxypropionate, beta-alanine synthesis via 3-hydroxypropionate Sources: GOC:mah, MetaCyc:PWY-3941 Relationships: is a type of beta-alanine biosynthetic process [GO:0019483]